{
  "gene": "UniProtKB:P49959",
  "term_id": "GO:0007095",
  "gene_symbol": "MRE11",
  "gene_name": "Double-strand break repair protein MRE11",
  "term_label": "mitotic G2 DNA damage checkpoint signaling"
}